{
  "term_label": "Unknown cellular component",
  "gene_name": "Endogenous retrovirus group S71 member 1 Env polyprotein",
  "gene_symbol": "ERVS71-1",
  "gene": "UniProtKB:P61550",
  "term_id": "UNKNOWN:0003"
}